GATOR1 complex [GO:1990130] (cellular component) References: PMID:21900499, PMID:23723238, PMID:23974112, PMID:25934700, PMID:28199306, PMID:29199950 Sources: GOC:krc, GOC:rb Definition: A GTPase-activating protein (GAP) complex that regulates TORC1 signaling by interacting with the Rag GTPase. In human, the GATOR1 complex consists of DEPDC5, NPRL2, and NPRL3. In S. cerevisiae, this complex is referred to as SEACIT and contains the Iml1p, Npr2p, and Npr3p proteins. Note: The Rag GTPase complex corresponds to Gtr1-Gtr2 GTPase complex ; GO:1990131. Relationships: is a type of protein-containing complex [GO:0032991]; is part of GO:0035859 Also known as: IML1 complex, SEACIT complex